regulation of Notch signaling pathway involved in somitogenesis [GO:1902366] (biological process) Relationships: is a type of GO:0008593; regulates Notch signaling pathway involved in somitogenesis [GO:1902359] Also known as: regulation of N signaling pathway involved in formation of mesodermal clusters, regulation of N signaling pathway involved in somitogenesis, regulation of N signalling pathway involved in formation of mesodermal clusters, regulation of N signalling pathway involved in somitogenesis, regulation of Notch receptor signaling pathway involved in formation of mesodermal clusters, regulation of Notch receptor signaling pathway involved in somitogenesis, regulation of Notch receptor signalling pathway involved in formation of mesodermal clusters, regulation of Notch receptor signalling pathway involved in somitogenesis, regulation of Notch signaling pathway involved in formation of mesodermal clusters, regulation of Notch signalling pathway involved in formation of mesodermal clusters, regulation of Notch signalling pathway involved in somitogenesis, regulation of Notch-receptor signaling pathway involved in formation of mesodermal clusters, regulation of Notch-receptor signaling pathway involved in somitogenesis, regulation of Notch-receptor signalling pathway involved in formation of mesodermal clusters, regulation of Notch-receptor signalling pathway involved in somitogenesis References: PMID:21795391 Sources: GOC:TermGenie, GOC:dph Definition: Any process that modulates the frequency, rate or extent of Notch signaling pathway involved in somitogenesis. Subtypes: negative regulation of Notch signaling pathway involved in somitogenesis [GO:1902367]